{
  "gene_name": "Probable global transcription activator SNF2L2",
  "term_label": "chromatin",
  "term_id": "GO:0000785",
  "gene_symbol": "SMARCA2",
  "gene": "UniProtKB:P51531"
}